activin A complex [GO:0043509] (cellular component) Relationships: is a type of activin complex [GO:0048180] Definition: A nonsteroidal regulator, composed of two covalently linked inhibin beta-A subunits (sometimes known as activin beta-A or activin/inhibin beta-A). Note: Note that the actions of the activin complex are the opposite of those of the inhibin complex, which is a dimer of an inhibin beta-A or inhibin beta-B subunit and an inhibin alpha subunit. See also the cellular component term 'inhibin complex ; GO:0043511'. Sources: GOC:go_curators